regulation of protein import into chloroplast stroma [GO:1904215] (biological process) Also known as: regulation of chloroplast stroma protein import, regulation of protein transport into chloroplast stroma References: PMID:25901327 Sources: GOC:TermGenie, GO_REF:0000058 Relationships: is a type of GO:0034762; is a type of regulation of protein transport [GO:0051223]; regulates GO:0045037 Subtypes: positive regulation of protein import into chloroplast stroma [GO:1904216] Definition: Any process that modulates the frequency, rate or extent of protein import into chloroplast stroma.